{
  "gene_name": "Zinc finger protein 33B",
  "term_id": "GO:0000122",
  "term_label": "negative regulation of transcription by RNA polymerase II",
  "gene": "UniProtKB:Q06732",
  "gene_symbol": "ZNF33B"
}